{
  "gene_symbol": "KRT27",
  "gene_name": "Keratin, type I cytoskeletal 27",
  "term_id": "GO:0030280",
  "term_label": "structural constituent of skin epidermis",
  "gene": "UniProtKB:Q7Z3Y8"
}